macromolecule depalmitoylation [GO:0098734] (biological process) Relationships: is a type of macromolecule deacylation [GO:0098732] Definition: The removal of palymitoyl groups from a macromolecule. Subtypes: protein depalmitoylation [GO:0002084] Sources: GOC:dos